T-helper 1 cell chemotaxis [GO:0035706] (biological process) Sources: CL:0000545, GOC:BHF Also known as: Th1 cell chemotaxis Definition: The directed movement of a T-helper 1 cell in response to an external stimulus. Relationships: is a type of T cell chemotaxis [GO:0010818]